{
  "term_label": "immunoglobulin mediated immune response",
  "gene_name": "Immunoglobulin heavy variable 1-58",
  "gene_symbol": "IGHV1-58",
  "gene": "UniProtKB:A0A0C4DH39",
  "term_id": "GO:0016064"
}